{
  "term_id": "UNKNOWN:0001",
  "gene_symbol": "LTBP3",
  "gene": "UniProtKB:Q9NS15",
  "term_label": "Unknown molecular function",
  "gene_name": "Latent-transforming growth factor beta-binding protein 3"
}